{
  "gene_symbol": "MON1A",
  "gene": "UniProtKB:Q86VX9",
  "term_label": "Unknown molecular function",
  "gene_name": "Vacuolar fusion protein MON1 homolog A",
  "term_id": "UNKNOWN:0001"
}